{
  "term_label": "cytoplasm",
  "gene": "UniProtKB:Q86YR7",
  "term_id": "GO:0005737",
  "gene_symbol": "MCF2L2",
  "gene_name": "Probable guanine nucleotide exchange factor MCF2L2"
}